PSII associated light-harvesting complex II binding [GO:0062066] (molecular function) Definition: Binding to a PSII associated light-harvesting complex II. References: PMID:17400553 Relationships: is_a protein-containing complex binding [GO:0044877]